{
  "gene_name": "5-hydroxytryptamine receptor 1D",
  "term_label": "dendrite",
  "gene_symbol": "HTR1D",
  "term_id": "GO:0030425",
  "gene": "UniProtKB:P28221"
}